negative regulation of anther dehiscence [GO:0120196] (biological process) Definition: Any process that stops, prevents, or reduces the frequency, rate or extent of anther dehiscence. References: PMID:30911018 Sources: GOC:lr Relationships: is a type of regulation of anther dehiscence [GO:0120194]; is a type of GO:2000242; negatively regulates anther dehiscence [GO:0009901]